{
  "gene_symbol": "CPTP",
  "gene": "UniProtKB:Q5TA50",
  "term_id": "GO:0005829",
  "term_label": "cytosol",
  "gene_name": "Ceramide-1-phosphate transfer protein"
}